malonate-semialdehyde dehydrogenase activity [GO:0033722] (MF) Also known as: 3-oxopropanoate:NAD(P)+ oxidoreductase activity, malonic semialdehyde dehydrogenase activity Definition: Catalysis of the reaction: 3-oxopropanoate + NAD(P)+ + H2O = malonate + NAD(P)H + H+. Relationships: is a type of oxidoreductase activity, acting on the aldehyde or oxo group of donors, NAD or NADP as acceptor [GO:0016620] Sources: EC:1.2.1.15